{
  "gene_symbol": "RASGRP4",
  "term_id": "GO:0005085",
  "term_label": "guanyl-nucleotide exchange factor activity",
  "gene": "UniProtKB:Q8TDF6",
  "gene_name": "RAS guanyl-releasing protein 4"
}